{
  "gene": "UniProtKB:Q99706",
  "term_id": "GO:0005886",
  "gene_name": "Killer cell immunoglobulin-like receptor 2DL4",
  "term_label": "plasma membrane",
  "gene_symbol": "KIR2DL4"
}